positive regulation of monoatomic ion transmembrane transport [GO:0034767] (biological process) Definition: Any process that activates or increases the frequency, rate or extent of the directed movement of ions from one side of a membrane to the other. Subtypes: positive regulation of ion transmembrane transporter activity [GO:0032414], positive regulation of anion transmembrane transport [GO:1903961], positive regulation of cation transmembrane transport [GO:1904064] Relationships: is a type of positive regulation of transmembrane transport [GO:0034764]; is a type of regulation of monoatomic ion transmembrane transport [GO:0034765]; is a type of positive regulation of monoatomic ion transport [GO:0043270]; positively regulates GO:0034220 Also known as: positive regulation of ion transmembrane transport, positive regulation of ion membrane transport, positive regulation of transmembrane ion transport, up regulation of transmembrane ion transport, up-regulation of transmembrane ion transport, upregulation of transmembrane ion transport, activation of transmembrane ion transport, stimulation of transmembrane ion transport Sources: GOC:mah